{
  "gene_name": "Motile sperm domain-containing protein 2",
  "term_label": "Unknown biological process",
  "term_id": "UNKNOWN:0002",
  "gene_symbol": "MOSPD2",
  "gene": "UniProtKB:Q8NHP6"
}